{
  "gene_name": "Centromere protein R",
  "term_label": "nucleoplasm",
  "gene_symbol": "ITGB3BP",
  "term_id": "GO:0005654",
  "gene": "UniProtKB:Q13352"
}